cellular response to prostaglandin I stimulus [GO:0071382] (biological process) Definition: Any process that results in a change in state or activity of a cell (in terms of movement, secretion, enzyme production, gene expression, etc.) as a result of a prostagladin I stimulus. Sources: GOC:mah Relationships: is a type of response to prostaglandin I [GO:0034697]; is a type of cellular response to prostaglandin stimulus [GO:0071379]; is a type of GO:1901701